regulation of cell migration involved in somitogenic axis elongation [GO:0090249] (biological process) Definition: Any process that modulates the frequency, rate, or extent of the controlled self-propelled movement of a cell that contributes to somitogenic axis elongation. Sources: GOC:ascb_2009, GOC:dph, GOC:tb Also known as: regulation of cell motility involved in somitogenic axis elongation Relationships: is a type of regulation of cell migration [GO:0030334]; regulates GO:0090248